{
  "gene_symbol": "RAB38",
  "gene": "UniProtKB:P57729",
  "term_id": "GO:0006886",
  "term_label": "intracellular protein transport",
  "gene_name": "Ras-related protein Rab-38"
}